{
  "gene": "UniProtKB:Q8TDG2",
  "gene_name": "Actin-related protein T1",
  "gene_symbol": "ACTRT1",
  "term_label": "actin cytoskeleton",
  "term_id": "GO:0015629"
}